{
  "term_id": "UNKNOWN:0001",
  "gene_symbol": "TMA16",
  "term_label": "Unknown molecular function",
  "gene": "UniProtKB:Q96EY4",
  "gene_name": "Translation machinery-associated protein 16"
}